oocyte maturation [GO:0001556] (biological process) Definition: A developmental process, independent of morphogenetic (shape) change, that is required for an oocyte to attain its fully functional state. Oocyte maturation commences after reinitiation of meiosis commonly starting with germinal vesicle breakdown, and continues up to the second meiotic arrest prior to fertilization. Relationships: is a type of GO:0003006; is a type of cell maturation [GO:0048469]; is part of GO:0048599 Regulation: regulated by regulation of oocyte maturation [GO:1900193]; negatively regulated by negative regulation of oocyte maturation [GO:1900194]; positively regulated by positive regulation of oocyte maturation [GO:1900195] Sources: GOC:devbiol, https://www.ncbi.nlm.nih.gov/books/NBK279054/